{
  "gene_symbol": "PAIP1",
  "term_label": "Unknown cellular component",
  "gene_name": "Polyadenylate-binding protein-interacting protein 1",
  "term_id": "UNKNOWN:0003",
  "gene": "UniProtKB:Q9H074"
}